{
  "gene_name": "ADP-ribosylation factor-binding protein GGA2",
  "gene_symbol": "GGA2",
  "gene": "UniProtKB:Q9UJY4",
  "term_id": "GO:0006893",
  "term_label": "Golgi to plasma membrane transport"
}